DNA binding, bending [GO:0008301] (molecular function) Relationships: is a type of DNA binding [GO:0003677] Subtypes: sequence-specific DNA binding, bending [GO:0044374], GO:0044378 Definition: The activity of binding selectively and non-covalently to and distorting the original structure of DNA, typically a straight helix, into a bend, or increasing the bend if the original structure was intrinsically bent due to its sequence. Also known as: DNA bending activity, DNA bending involving DNA binding References: PMID:10710711, PMID:19037758 Sources: GOC:krc, GOC:vw